dihydropteridine metabolic process [GO:0051067] (biological process) Relationships: is a type of pteridine-containing compound metabolic process [GO:0042558] References: PMID:2557335 Definition: The chemical reactions and pathways involving 6,7-dihydropteridine, a bicyclic compound with the formula C6H6N4. Also known as: 6,7-dihydropteridine metabolic process, dihydropteridine metabolism, dihydropteridine reduction